trans-synaptic protein complex [GO:0098820] (cellular component) Definition: A protein complex that spans the synaptic cleft and has parts in both the pre- and post-synaptic membranes. References: PMID:20200227 Relationships: is a type of GO:0032991